{
  "gene_symbol": "C5AR2",
  "gene": "UniProtKB:Q9P296",
  "gene_name": "C5a anaphylatoxin chemotactic receptor 2",
  "term_label": "G protein-coupled receptor activity",
  "term_id": "GO:0004930"
}